{
  "term_label": "activin receptor activity",
  "gene": "UniProtKB:Q13705",
  "term_id": "GO:0017002",
  "gene_symbol": "ACVR2B",
  "gene_name": "Activin receptor type-2B"
}